{
  "gene_symbol": "LIMS1",
  "gene_name": "LIM and senescent cell antigen-like-containing domain protein 1",
  "term_label": "Unknown molecular function",
  "term_id": "UNKNOWN:0001",
  "gene": "UniProtKB:P48059"
}